{
  "term_id": "UNKNOWN:0001",
  "gene_symbol": "C2",
  "term_label": "Unknown molecular function",
  "gene": "UniProtKB:P06681",
  "gene_name": "Complement C2"
}